{
  "term_id": "UNKNOWN:0003",
  "gene_name": "Pleckstrin homology domain-containing family G member 6",
  "term_label": "Unknown cellular component",
  "gene": "UniProtKB:Q3KR16",
  "gene_symbol": "PLEKHG6"
}